RNA polymerase III type 3 promoter sequence-specific DNA binding [GO:0001006] (molecular function) References: PMID:12381659 Sources: GOC:txnOH Also known as: RNA polymerase III type 3 promoter DNA binding Definition: Binding to a sequence of DNA that is a part of a type 3 promoter that controls transcription by RNA polymerase III (Pol III). A type 3 Pol III promoter is composed of elements upstream of the transcription start site, including a TATA box. The human U6 snRNA gene has a type 3 promoter. Type 3 Pol III promoters have not been observed in S. cerevisiae. Relationships: is a type of GO:0000992